{
  "term_label": "positive regulation of cholesterol efflux",
  "gene": "UniProtKB:P55055",
  "term_id": "GO:0010875",
  "gene_symbol": "NR1H2",
  "gene_name": "Oxysterols receptor LXR-beta"
}